bacterial thylakoid [GO:0030075] (cellular component) Also known as: plasma membrane-derived thylakoid Definition: A thylakoid that is derived from and attached to, but not necessarily continuous with, the plasma membrane, and is not enclosed in a plastid. It bears the photosynthetic pigments in photosynthetic cyanobacteria. Sources: GOC:mah, GOC:mtg_sensu Relationships: is a type of GO:0009579